negative regulation of development, heterochronic [GO:0045961] (BP) Also known as: down regulation of development, heterochronic, down-regulation of development, heterochronic, downregulation of development, heterochronic, inhibition of development, heterochronic Sources: GOC:go_curators Definition: Any process that modulates the consistent predetermined time point at which an integrated living unit or organism progresses from an initial condition to a later condition and decreases the rate at which this time point is reached. Relationships: is a type of regulation of development, heterochronic [GO:0040034] Subtypes: negative regulation of nematode larval development, heterochronic [GO:0090446]